{
  "term_id": "GO:0003677",
  "term_label": "DNA binding",
  "gene_name": "Chromodomain-helicase-DNA-binding protein 2",
  "gene_symbol": "CHD2",
  "gene": "UniProtKB:O14647"
}